{
  "gene_symbol": "JAZF1",
  "gene_name": "Juxtaposed with another zinc finger protein 1",
  "gene": "UniProtKB:Q86VZ6",
  "term_id": "UNKNOWN:0001",
  "term_label": "Unknown molecular function"
}